{
  "term_id": "GO:0008017",
  "term_label": "microtubule binding",
  "gene": "UniProtKB:Q6ZMV9",
  "gene_name": "Kinesin-like protein KIF6",
  "gene_symbol": "KIF6"
}